myotube differentiation involved in skeletal muscle regeneration [GO:0014908] (biological process) Sources: GOC:mtg_muscle Definition: The process in which a relatively unspecialized cell acquires specialized features of a myotube cell. Myotube differentiation starts with myoblast fusion and the appearance of specific cell markers (this is the cell development step). Then individual myotubes can fuse to form bigger myotubes and start to contract. This process occurs as part of the process of skeletal muscle regeneration. Myotubes are multinucleated cells that are formed when proliferating myoblasts exit the cell cycle, differentiate and fuse. Relationships: is a type of GO:0014902; BFO_0000050 skeletal muscle tissue regeneration [GO:0043403]